rhombomere formation [GO:0021594] (biological process) Sources: GOC:cls, GOC:dgh, GOC:dph, GOC:jid, GO_REF:0000021 Relationships: is a type of anatomical structure formation involved in morphogenesis [GO:0048646]; is part of rhombomere morphogenesis [GO:0021593] Definition: The process that gives rise to the rhombomere. This process pertains to the initial formation of a structure from unspecified parts. Rhombomeres are transverse segments of the developing rhombencephalon. Rhombomeres are lineage restricted, express different genes from one another, and adopt different developmental fates. Subtypes: rhombomere 1 formation [GO:0021652], GO:0021657, rhombomere 3 formation [GO:0021660], rhombomere 4 formation [GO:0021663], GO:0021666, GO:0021669, rhombomere 7 formation [GO:0021673], rhombomere 8 formation [GO:0021677]